{
  "term_id": "GO:0046628",
  "term_label": "positive regulation of insulin receptor signaling pathway",
  "gene_name": "Erythroferrone",
  "gene_symbol": "ERFE",
  "gene": "UniProtKB:Q4G0M1"
}